aldehyde dehydrogenase (FAD-independent) activity [GO:0033727] (molecular function) Definition: Catalysis of the reaction: an aldehyde + H2O + acceptor = a carboxylate + reduced acceptor. Also known as: AORDd, Mop, aldehyde oxidoreductase activity, aldehyde:acceptor oxidoreductase (FAD-independent) activity Sources: EC:1.2.99.7 Relationships: is a type of GO:0016903